{
  "term_label": "negative regulation of double-strand break repair via homologous recombination",
  "term_id": "GO:2000042",
  "gene": "UniProtKB:Q8N884",
  "gene_name": "Cyclic GMP-AMP synthase",
  "gene_symbol": "CGAS"
}